{
  "gene_symbol": "SHROOM2",
  "term_id": "GO:0007015",
  "term_label": "actin filament organization",
  "gene_name": "Protein Shroom2",
  "gene": "UniProtKB:Q13796"
}